{
  "gene_name": "Serine_threonine-protein kinase_endoribonuclease IRE2",
  "gene": "UniProtKB:Q76MJ5",
  "gene_symbol": "ERN2",
  "term_id": "GO:1990604",
  "term_label": "IRE1-TRAF2-ASK1 complex"
}